isoquinoline alkaloid biosynthetic process [GO:0033075] (biological process) Relationships: is a type of alkaloid biosynthetic process [GO:0009821]; is a type of isoquinoline alkaloid metabolic process [GO:0033076] Also known as: isoquinoline alkaloid anabolism, isoquinoline alkaloid biosynthesis, isoquinoline alkaloid formation, isoquinoline alkaloid synthesis, ipecac alkaloid biosynthesis Definition: The chemical reactions and pathways resulting in the formation of isoquinoline alkaloids, alkaloid compounds that contain bicyclic N-containing aromatic rings and are derived from a 3,4-dihydroxytyramine (dopamine) precursor that undergoes a Schiff base addition with aldehydes of different origin. Subtypes: benzyl isoquinoline alkaloid biosynthetic process [GO:0009708], GO:0035831, morphine biosynthetic process [GO:0097295], (S)-scoulerine biosynthetic process [GO:1901009] References: PMID:26503307 Sources: GOC:mah